{
  "gene_symbol": "KIF21A",
  "term_label": "cytoplasm",
  "term_id": "GO:0005737",
  "gene_name": "Kinesin-like protein KIF21A",
  "gene": "UniProtKB:Q7Z4S6"
}